{
  "term_id": "GO:0032869",
  "term_label": "cellular response to insulin stimulus",
  "gene_name": "Insulin-induced gene 2 protein",
  "gene_symbol": "INSIG2",
  "gene": "UniProtKB:Q9Y5U4"
}